{
  "gene_symbol": "HELB",
  "gene": "UniProtKB:Q8NG08",
  "gene_name": "DNA helicase B",
  "term_label": "5'-3' DNA helicase activity",
  "term_id": "GO:0043139"
}